{
  "gene": "UniProtKB:Q86VK4",
  "term_id": "GO:0005634",
  "term_label": "nucleus",
  "gene_symbol": "ZNF410",
  "gene_name": "Zinc finger protein 410"
}